{
  "gene_symbol": "SPDEF",
  "gene": "UniProtKB:O95238",
  "gene_name": "SAM pointed domain-containing Ets transcription factor",
  "term_label": "nucleus",
  "term_id": "GO:0005634"
}